natural killer cell chemotaxis [GO:0035747] (biological process) Regulation: regulated by regulation of natural killer cell chemotaxis [GO:2000501]; negatively regulated by GO:2000502; positively regulated by positive regulation of natural killer cell chemotaxis [GO:2000503] Sources: CL:0000623, GOC:BHF Definition: The directed movement of a natural killer cell guided by a specific chemical concentration gradient. Movement may be towards a higher concentration (positive chemotaxis) or towards a lower concentration (negative chemotaxis). Relationships: is a type of lymphocyte chemotaxis [GO:0048247] Subtypes: mature natural killer cell chemotaxis [GO:0035782]